{
  "gene": "UniProtKB:P0C7X3",
  "gene_name": "Putative cyclin-Y-like protein 3",
  "gene_symbol": "CCNYL3",
  "term_id": "GO:0061575",
  "term_label": "cyclin-dependent protein serine/threonine kinase activator activity"
}